taurine catabolic process [GO:0019529] (biological process) Definition: The chemical reactions and pathways resulting in the breakdown of taurine (2-aminoethanesulfonic acid), a sulphur-containing amino acid derivative important in the metabolism of fats. Relationships: is a type of GO:0019530; is a type of alkanesulfonate catabolic process [GO:0046306] Sources: GOC:jl, ISBN:0198600461 Also known as: taurine breakdown, taurine catabolism, taurine degradation